{
  "gene_symbol": "DHX35",
  "term_label": "catalytic step 2 spliceosome",
  "gene_name": "Probable ATP-dependent RNA helicase DHX35",
  "gene": "UniProtKB:Q9H5Z1",
  "term_id": "GO:0071013"
}